{
  "gene_symbol": "TMPRSS3",
  "term_id": "GO:0007605",
  "gene": "UniProtKB:P57727",
  "gene_name": "Transmembrane protease serine 3",
  "term_label": "sensory perception of sound"
}